{
  "term_label": "Unknown molecular function",
  "term_id": "UNKNOWN:0001",
  "gene_name": "Fibrosin-1-like protein",
  "gene_symbol": "FBRSL1",
  "gene": "UniProtKB:Q9HCM7"
}